{
  "gene": "UniProtKB:Q14651",
  "gene_name": "Plastin-1",
  "gene_symbol": "PLS1",
  "term_id": "GO:0005737",
  "term_label": "cytoplasm"
}